{
  "gene_symbol": "FIP1L1",
  "gene": "UniProtKB:Q6UN15",
  "gene_name": "Pre-mRNA 3'-end-processing factor FIP1",
  "term_id": "GO:0006398",
  "term_label": "mRNA 3'-end processing by stem-loop binding and cleavage"
}